U4atac snRNP [GO:0005690] (cellular component) Also known as: snRNP U4atac Definition: A ribonucleoprotein complex that contains small nuclear RNA U4atac, a heptameric ring of Sm proteins, as well as several proteins that are unique to the U4atac snRNP, most of which remain associated with the U4atac snRNA both while the U4atac snRNP is free or assembled into the U4atac/U6atac complex or into a series of spliceosomal complexes. Relationships: is a type of spliceosomal snRNP complex [GO:0097525] Sources: GOC:krc, GOC:mah, ISBN:0879695897